glutamic-type endopeptidase activity [GO:0070007] (molecular function) Definition: Catalysis of the hydrolysis of internal peptide bonds in a polypeptide chain by a mechanism involving a glutamate/glutamine catalytic dyad. Sources: GOC:mah, https://www.ebi.ac.uk/merops/about/glossary.shtml#CATTYPE, https://www.ebi.ac.uk/merops/about/glossary.shtml#ENDOPEPTIDASE Relationships: is a type of endopeptidase activity [GO:0004175]; is a type of glutamic-type peptidase activity [GO:0070002]